{
  "gene": "UniProtKB:P80511",
  "term_id": "GO:0061844",
  "gene_symbol": "S100A12",
  "term_label": "antimicrobial humoral immune response mediated by antimicrobial peptide",
  "gene_name": "Protein S100-A12"
}